{
  "term_label": "phospholipid translocation",
  "term_id": "GO:0045332",
  "gene_symbol": "ATP8A2",
  "gene_name": "Phospholipid-transporting ATPase IB",
  "gene": "UniProtKB:Q9NTI2"
}